negative regulation of necroptotic process [GO:0060546] (biological process) Also known as: negative regulation of necroptosis Relationships: is a type of regulation of necroptotic process [GO:0060544]; is a type of negative regulation of programmed necrotic cell death [GO:0062099]; negatively regulates necroptotic process [GO:0070266] Sources: GOC:BHF, GOC:dph, GOC:mtg_apoptosis, GOC:tb Definition: Any process that decreases the rate, frequency or extent of a necroptotic process, a necrotic cell death process that results from the activation of endogenous cellular processes, such as signaling involving death domain receptors or Toll-like receptors.